telomerase RNA stabilization [GO:0090669] (BP) Definition: Prevention of degradation of telomerase RNA (TERC) molecules. Relationships: is a type of RNA stabilization [GO:0043489] References: PMID:25467444 Sources: GOC:BHF, GOC:BHF_telomere, GOC:nc Also known as: TERC stabilization